{
  "gene_symbol": "CHMP4A",
  "gene_name": "Charged multivesicular body protein 4a",
  "gene": "UniProtKB:Q9BY43",
  "term_id": "GO:0005635",
  "term_label": "nuclear envelope"
}